{
  "gene": "UniProtKB:P10147",
  "gene_symbol": "CCL3",
  "gene_name": "C-C motif chemokine 3",
  "term_id": "GO:0060326",
  "term_label": "cell chemotaxis"
}